{
  "term_label": "Unknown molecular function",
  "gene_symbol": "TEX19",
  "gene_name": "Testis-expressed protein 19",
  "gene": "UniProtKB:Q8NA77",
  "term_id": "UNKNOWN:0001"
}